methanogenesis, from carbon dioxide [GO:0019386] (BP) Relationships: is a type of methanogenesis [GO:0015948] Definition: The chemical reactions and pathways resulting in the formation of methane, a colorless, odorless, flammable gas with the formula CH4, from other compounds, including carbon dioxide (CO2). Sources: GOC:ai Also known as: methane biosynthesis from carbon dioxide, methane biosynthetic process from carbon dioxide